regulation of melanization defense response [GO:0035007] (biological process) Subtypes: positive regulation of melanization defense response [GO:0035008], GO:0035009, regulation of melanotic encapsulation of foreign target [GO:0140539] Sources: GOC:bf Definition: Any process that affects the rate, extent or location of the melanization defense response during injury or invasion. Also known as: regulation of melanization defence response Relationships: is a type of GO:0043455; is a type of regulation of innate immune response [GO:0045088]; regulates GO:0035006